{
  "term_id": "UNKNOWN:0001",
  "gene": "UniProtKB:Q6ZUT3",
  "gene_symbol": "FRMD7",
  "term_label": "Unknown molecular function",
  "gene_name": "FERM domain-containing protein 7"
}